{
  "gene_symbol": "KNL1",
  "term_label": "protein localization to kinetochore",
  "gene_name": "Kinetochore scaffold 1",
  "gene": "UniProtKB:Q8NG31",
  "term_id": "GO:0034501"
}